{
  "term_label": "nucleus",
  "gene_symbol": "FBXO5",
  "term_id": "GO:0005634",
  "gene_name": "F-box only protein 5",
  "gene": "UniProtKB:Q9UKT4"
}